{
  "gene_symbol": "PALM",
  "gene": "UniProtKB:O75781",
  "term_id": "GO:0044309",
  "gene_name": "Paralemmin-1",
  "term_label": "neuron spine"
}